organellar large ribosomal subunit [GO:0000315] (cellular component) Definition: The larger of the two subunits of an organellar ribosome. Two sites on the ribosomal large subunit are involved in translation: the aminoacyl site (A site) and peptidyl site (P site). Subtypes: plastid large ribosomal subunit [GO:0000311], mitochondrial large ribosomal subunit [GO:0005762] Relationships: is a type of large ribosomal subunit [GO:0015934]; BFO_0000050 organellar ribosome [GO:0000313] Sources: GOC:mcc